protein ubiquitination [GO:0016567] (biological process) References: PMID:26906419 Regulation: regulated by regulation of protein ubiquitination [GO:0031396]; negatively regulated by negative regulation of protein ubiquitination [GO:0031397]; positively regulated by positive regulation of protein ubiquitination [GO:0031398] Definition: The process in which one or more ubiquitin groups are added to a protein. Also known as: protein ubiquitinylation, protein ubiquitylation Relationships: is a type of GO:0032446 Subtypes: protein polyubiquitination [GO:0000209], protein monoubiquitination [GO:0006513], GO:0007014, protein autoubiquitination [GO:0051865]